{
  "gene_symbol": "FAM218A",
  "term_id": "UNKNOWN:0001",
  "term_label": "Unknown molecular function",
  "gene_name": "Protein FAM218A",
  "gene": "UniProtKB:Q96MZ4"
}